{
  "term_id": "GO:0030574",
  "term_label": "collagen catabolic process",
  "gene_name": "Matrix metalloproteinase-20",
  "gene": "UniProtKB:O60882",
  "gene_symbol": "MMP20"
}